{
  "gene_symbol": "MMP16",
  "gene_name": "Matrix metalloproteinase-16",
  "term_label": "collagen catabolic process",
  "term_id": "GO:0030574",
  "gene": "UniProtKB:P51512"
}